{
  "gene_symbol": "SLC5A3",
  "term_label": "plasma membrane",
  "term_id": "GO:0005886",
  "gene_name": "Sodium_myo-inositol cotransporter",
  "gene": "UniProtKB:P53794"
}